{
  "gene": "UniProtKB:Q2Q1W2",
  "gene_name": "E3 ubiquitin-protein ligase TRIM71",
  "term_id": "GO:0035198",
  "gene_symbol": "TRIM71",
  "term_label": "miRNA binding"
}